{
  "gene_name": "Keratin-associated protein 21-3",
  "gene_symbol": "KRTAP21-3",
  "gene": "UniProtKB:Q3LHN1",
  "term_id": "UNKNOWN:0003",
  "term_label": "Unknown cellular component"
}